{
  "term_label": "Unknown molecular function",
  "gene_name": "Immunoglobulin kappa variable 1D-8",
  "gene": "UniProtKB:A0A087WSZ0",
  "term_id": "UNKNOWN:0001",
  "gene_symbol": "IGKV1D-8"
}